{
  "gene_name": "Saccharopine dehydrogenase-like oxidoreductase",
  "term_label": "glycolipid biosynthetic process",
  "term_id": "GO:0009247",
  "gene_symbol": "SCCPDH",
  "gene": "UniProtKB:Q8NBX0"
}